{
  "term_id": "GO:0035567",
  "gene": "UniProtKB:Q9H461",
  "gene_name": "Frizzled-8",
  "term_label": "non-canonical Wnt signaling pathway",
  "gene_symbol": "FZD8"
}